{
  "gene": "UniProtKB:Q8NI35",
  "gene_name": "InaD-like protein",
  "term_label": "cytoplasm",
  "term_id": "GO:0005737",
  "gene_symbol": "PATJ"
}